membrane destabilizing activity [GO:0140912] (molecular function) References: PMID:34496967 Relationships: is a type of GO:0003674 Also known as: antimicrobial peptide Definition: Binding to a membrane and increasing its permeability. This may lead to cell membrane lysis and cell content release.